regulation of protein kinase activity [GO:0045859] (biological process) Sources: GOC:go_curators Definition: Any process that modulates the frequency, rate or extent of protein kinase activity. Relationships: is a type of regulation of protein phosphorylation [GO:0001932]; is a type of regulation of kinase activity [GO:0043549]; regulates GO:0004672 Subtypes: negative regulation of protein kinase activity [GO:0006469], GO:0045860, regulation of protein tyrosine kinase activity [GO:0061097], regulation of protein serine/threonine kinase activity [GO:0071900]